{
  "gene_name": "Gap junction alpha-5 protein",
  "gene_symbol": "GJA5",
  "gene": "UniProtKB:P36382",
  "term_id": "GO:0007267",
  "term_label": "cell-cell signaling"
}